{
  "term_label": "Unknown molecular function",
  "gene_name": "DDB1- and CUL4-associated factor 16",
  "gene": "UniProtKB:Q9NXF7",
  "term_id": "UNKNOWN:0001",
  "gene_symbol": "DCAF16"
}